regulation of antifungal peptide biosynthetic process [GO:0002810] (biological process) Definition: Any process that modulates the frequency, rate, or extent of antifungal peptide biosynthesis. Sources: GOC:add Subtypes: negative regulation of antifungal peptide biosynthetic process [GO:0002811], positive regulation of antifungal peptide biosynthetic process [GO:0006967] Relationships: is a type of regulation of antifungal peptide production [GO:0002788]; is a type of GO:0002805; regulates antifungal peptide biosynthetic process [GO:0002783]